{
  "gene_symbol": "PCP2",
  "gene_name": "Purkinje cell protein 2 homolog",
  "gene": "UniProtKB:Q8IVA1",
  "term_id": "UNKNOWN:0002",
  "term_label": "Unknown biological process"
}